{
  "gene": "UniProtKB:Q96DT5",
  "term_id": "GO:0030286",
  "gene_name": "Dynein axonemal heavy chain 11",
  "gene_symbol": "DNAH11",
  "term_label": "dynein complex"
}